{
  "gene_symbol": "PGAM5",
  "gene": "UniProtKB:Q96HS1",
  "term_label": "mitochondrion",
  "gene_name": "Serine_threonine-protein phosphatase PGAM5, mitochondrial",
  "term_id": "GO:0005739"
}